{
  "term_id": "GO:0048786",
  "gene_name": "Liprin-alpha-1",
  "gene_symbol": "PPFIA1",
  "term_label": "presynaptic active zone",
  "gene": "UniProtKB:Q13136"
}